{
  "term_id": "GO:0043066",
  "gene_name": "Transcription factor AP-2-beta",
  "gene_symbol": "TFAP2B",
  "gene": "UniProtKB:Q92481",
  "term_label": "negative regulation of apoptotic process"
}